{
  "term_label": "olfactory receptor activity",
  "gene_symbol": "OR10A2",
  "term_id": "GO:0004984",
  "gene": "UniProtKB:Q9H208",
  "gene_name": "Olfactory receptor 10A2"
}